{
  "gene_symbol": "ATP2A1",
  "gene_name": "Sarcoplasmic_endoplasmic reticulum calcium ATPase 1",
  "gene": "UniProtKB:O14983",
  "term_id": "GO:0006874",
  "term_label": "intracellular calcium ion homeostasis"
}